regulation of chlorophyll catabolic process [GO:0010271] (biological process) Definition: Any process that modulates the frequency, rate or extent of the chemical reactions and pathways resulting in the breakdown of chlorophyll. References: PMID:16361392 Relationships: is_a GO:0090056; is a type of regulation of tetrapyrrole catabolic process [GO:1901404]; regulates chlorophyll catabolic process [GO:0015996] Subtypes: GO:1903647, GO:1903648